methylselenol reductase activity [GO:0098625] (MF) References: PMID:11782468 Relationships: is a type of oxidoreductase activity, acting on NAD(P)H [GO:0016651] Definition: Catalysis of the reaction: NADPH + H+ + CH3SeOH = NADP+ + CH3SeH + H2O.